{
  "term_id": "GO:0001540",
  "gene_name": "Amyloid beta precursor protein binding family B member 1",
  "term_label": "amyloid-beta binding",
  "gene_symbol": "APBB1",
  "gene": "UniProtKB:O00213"
}